{
  "term_id": "UNKNOWN:0001",
  "gene_symbol": "C16orf54",
  "gene_name": "Transmembrane protein C16orf54",
  "gene": "UniProtKB:Q6UWD8",
  "term_label": "Unknown molecular function"
}